hippocampal mossy fiber to CA3 synapse [GO:0098686] (cellular component) Relationships: is a type of neuron to neuron synapse [GO:0098984]; has part GO:0097464; has part hippocampal mossy fiber expansion [GO:1990026] Definition: One of the giant synapses that form between the mossy fiber axons of dentate gyrus granule cells and the large complex spines of CA3 pyramidal cells. It consists of a giant bouton known as the mossy fiber expansion, synapsed to the complex, multiheaded spine (thorny excresence) of a CA3 pyramidal cell. References: PMID:13869693, PMID:23264762 Sources: DOI:10.1002/1096-9861